{
  "term_label": "adenylate cyclase-activating dopamine receptor signaling pathway",
  "gene_symbol": "GNAS",
  "gene": "UniProtKB:Q5JWF2",
  "gene_name": "Guanine nucleotide-binding protein G(s) subunit alpha isoforms XLas",
  "term_id": "GO:0007191"
}